{
  "term_id": "GO:0005509",
  "gene": "UniProtKB:Q86SJ6",
  "term_label": "calcium ion binding",
  "gene_name": "Desmoglein-4",
  "gene_symbol": "DSG4"
}